antifungal peptide production [GO:0002781] (biological process) Relationships: is a type of GO:0002775; is part of GO:0019732 Definition: The synthesis or release of an antifungal peptide during an immune response, resulting in an increase in intracellular or extracellular levels. References: PMID:11807545, PMID:15638771 Sources: GOC:add, ISBN:0781735149 Regulation: RO_0002211 by regulation of antifungal peptide production [GO:0002788]; negatively regulated by GO:0002789; positively regulated by GO:0002804 Note: Note that this term is in the subset of terms that should not be used for direct gene product annotation. Instead, select one of the 'regulation' children terms.